{
  "gene": "UniProtKB:Q9UHD0",
  "gene_symbol": "IL19",
  "term_id": "GO:0005615",
  "gene_name": "Interleukin-19",
  "term_label": "extracellular space"
}